{
  "term_label": "synapse",
  "gene_name": "Cell adhesion molecule 1",
  "term_id": "GO:0045202",
  "gene": "UniProtKB:Q9BY67",
  "gene_symbol": "CADM1"
}